{
  "gene_name": "Zinc transporter ZIP3",
  "gene": "UniProtKB:Q9BRY0",
  "term_id": "GO:0005385",
  "term_label": "zinc ion transmembrane transporter activity",
  "gene_symbol": "SLC39A3"
}